{
  "gene_symbol": "FGF9",
  "term_id": "GO:0030334",
  "term_label": "regulation of cell migration",
  "gene": "UniProtKB:P31371",
  "gene_name": "Fibroblast growth factor 9"
}